{
  "gene_name": "Desmocollin-1",
  "term_label": "cell-cell adhesion",
  "gene_symbol": "DSC1",
  "term_id": "GO:0098609",
  "gene": "UniProtKB:Q08554"
}